{
  "term_label": "DNA-binding transcription factor activity, RNA polymerase II-specific",
  "gene": "UniProtKB:Q5SQQ9",
  "term_id": "GO:0000981",
  "gene_name": "Ventral anterior homeobox 1",
  "gene_symbol": "VAX1"
}